{
  "gene_name": "5-demethoxyubiquinone hydroxylase, mitochondrial",
  "term_label": "regulation of reactive oxygen species metabolic process",
  "gene": "UniProtKB:Q99807",
  "gene_symbol": "COQ7",
  "term_id": "GO:2000377"
}